molybdenum ion transmembrane transporter activity [GO:0042888] (molecular function) Relationships: is_a GO:0046915 Definition: Enables the transfer of molybdenum (Mo) ions from one side of a membrane to the other. Sources: GOC:jl, ISBN:0198506732